{
  "term_id": "UNKNOWN:0001",
  "gene": "UniProtKB:Q5T7W7",
  "gene_name": "Thiosulfate sulfurtransferase_rhodanese-like domain-containing protein 2",
  "term_label": "Unknown molecular function",
  "gene_symbol": "TSTD2"
}